{
  "gene_symbol": "FLCN",
  "gene": "UniProtKB:Q8NFG4",
  "term_label": "Unknown molecular function",
  "term_id": "UNKNOWN:0001",
  "gene_name": "Folliculin"
}